{
  "gene_symbol": "EPHA3",
  "term_label": "ephrin receptor signaling pathway",
  "gene_name": "Ephrin type-A receptor 3",
  "term_id": "GO:0048013",
  "gene": "UniProtKB:P29320"
}